{
  "gene_name": "Laminin subunit gamma-1",
  "term_id": "GO:0005201",
  "term_label": "extracellular matrix structural constituent",
  "gene": "UniProtKB:P11047",
  "gene_symbol": "LAMC1"
}